{
  "term_label": "negative regulation of cell migration",
  "gene_name": "SLIT-ROBO Rho GTPase-activating protein 1",
  "gene": "UniProtKB:Q7Z6B7",
  "term_id": "GO:0030336",
  "gene_symbol": "SRGAP1"
}